{
  "term_id": "UNKNOWN:0001",
  "gene_symbol": "IL1RAPL1",
  "gene": "UniProtKB:Q9NZN1",
  "term_label": "Unknown molecular function",
  "gene_name": "Interleukin-1 receptor accessory protein-like 1"
}